arabinosyltransferase activity [GO:0052636] (molecular function) Definition: Catalysis of the transfer of an arabinosyl group from one compound (donor) to another (acceptor). Sources: GOC:ai Subtypes: indolylacetylinositol arabinosyltransferase activity [GO:0050409], flavonol 3-O-arabinosyltransferase activity [GO:0080059] Relationships: is_a pentosyltransferase activity [GO:0016763] Also known as: arabinosyl transferase activity